{
  "gene_name": "Pituitary tumor-transforming gene 1 protein-interacting protein",
  "term_label": "Unknown molecular function",
  "term_id": "UNKNOWN:0001",
  "gene_symbol": "PTTG1IP",
  "gene": "UniProtKB:P53801"
}